{
  "term_label": "mitotic spindle astral microtubule",
  "gene": "UniProtKB:Q86Y91",
  "gene_name": "Kinesin-like protein KIF18B",
  "gene_symbol": "KIF18B",
  "term_id": "GO:0061673"
}